{
  "gene_symbol": "ADCY10",
  "term_label": "Unknown biological process",
  "gene_name": "Adenylate cyclase type 10",
  "term_id": "UNKNOWN:0002",
  "gene": "UniProtKB:Q96PN6"
}